symbiont-mediated suppression of host DNA replication [GO:0098673] (biological process) Definition: Any process by which a virus inhibits DNA replication in its host cell. Some bacteriophages are known to do this, possibly as a way of increasing the pool of nucleotides available for virus replication. References: PMID:17010157, PMID:21205014 Also known as: inhibition of host DNA replication by virus Relationships: is_a symbiont-mediated perturbation of host cellular process [GO:0044068]